{
  "gene_name": "Cytosolic purine 5'-nucleotidase",
  "gene_symbol": "NT5C2",
  "gene": "UniProtKB:P49902",
  "term_id": "GO:0046040",
  "term_label": "IMP metabolic process"
}